regulation of initiation of mating projection growth [GO:0031384] (biological process) Definition: Any process that modulates the frequency, rate, or extent of the start of mating projection formation by unicellular fungi. Relationships: is a type of regulation of mating projection assembly [GO:0031383] References: PMID:14734532